{
  "term_id": "UNKNOWN:0001",
  "term_label": "Unknown molecular function",
  "gene_name": "Aminoacyl tRNA synthase complex-interacting multifunctional protein 2",
  "gene_symbol": "AIMP2",
  "gene": "UniProtKB:Q13155"
}